{
  "gene_name": "Major facilitator superfamily domain-containing protein 4A",
  "term_label": "Unknown cellular component",
  "gene": "UniProtKB:Q8N468",
  "gene_symbol": "MFSD4A",
  "term_id": "UNKNOWN:0003"
}